{
  "gene_name": "Leucine-rich repeat-containing protein 37B",
  "gene_symbol": "LRRC37B",
  "term_label": "Unknown molecular function",
  "term_id": "UNKNOWN:0001",
  "gene": "UniProtKB:Q96QE4"
}